plant-type cell wall modification [GO:0009827] (biological process) Sources: GOC:lr, GOC:mtg_sensu Also known as: cellulose and pectin-containing cell wall modification Subtypes: plant-type cell wall loosening [GO:0009828], GO:0009829, GO:0009830, GO:0009831, GO:1905588 Relationships: is a type of GO:0009664; is a type of cell wall modification [GO:0042545] Definition: The series of events leading to chemical and structural alterations of an existing cellulose and pectin-containing cell wall that can result in loosening, increased extensibility or disassembly. An example of this is found in Arabidopsis thaliana.